{
  "gene_name": "Scaffold attachment factor B1",
  "term_label": "estrogen receptor signaling pathway",
  "gene": "UniProtKB:Q15424",
  "gene_symbol": "SAFB",
  "term_id": "GO:0030520"
}